{
  "gene_name": "Zinc finger protein 1 homolog",
  "gene": "UniProtKB:Q6P2D0",
  "gene_symbol": "ZFP1",
  "term_label": "regulation of transcription by RNA polymerase II",
  "term_id": "GO:0006357"
}